regulation of translation at synapse [GO:0140243] (biological process) Note: Note that this term was created for the SynGO project, and will be obsoleted when the SynGO annotations are made in Noctua. Definition: Any process that regulates translation occurring at the synapse. References: PMID:20427644 Subtypes: regulation of translation at synapse, modulating synaptic transmission [GO:0099547], regulation of translation at presynapse [GO:0140244], GO:0140245 Relationships: is a type of GO:0006417; occurs in synapse [GO:0045202]